{
  "gene_name": "Sodium channel subunit beta-3",
  "gene_symbol": "SCN3B",
  "gene": "UniProtKB:Q9NY72",
  "term_label": "sodium channel inhibitor activity",
  "term_id": "GO:0019871"
}